{
  "term_label": "plasma membrane",
  "term_id": "GO:0005886",
  "gene_name": "Melanin-concentrating hormone receptor 2",
  "gene_symbol": "MCHR2",
  "gene": "UniProtKB:Q969V1"
}